{
  "gene_symbol": "WNT2B",
  "term_id": "GO:0030182",
  "gene": "UniProtKB:Q93097",
  "term_label": "neuron differentiation",
  "gene_name": "Protein Wnt-2b"
}